{
  "gene_symbol": "NKX2-8",
  "term_id": "GO:0006357",
  "term_label": "regulation of transcription by RNA polymerase II",
  "gene": "UniProtKB:O15522",
  "gene_name": "Homeobox protein Nkx-2.8"
}